cinnamic acid catabolic process [GO:0046281] (biological process) Definition: The chemical reactions and pathways resulting in the breakdown of cinnamic acid, 3-phenyl-2-propenoic acid. Sources: GOC:ai Also known as: cinnamic acid breakdown, cinnamic acid catabolism, cinnamic acid degradation, cinnamylic acid catabolic process, cinnamylic acid catabolism, phenylacrylic acid catabolic process, phenylacrylic acid catabolism Relationships: is a type of cinnamic acid metabolic process [GO:0009803]; is_a phenylpropanoid catabolic process [GO:0046271]; is a type of monocarboxylic acid catabolic process [GO:0072329]; is a type of olefinic compound catabolic process [GO:0120256]